{
  "gene_symbol": "NUTM2E",
  "gene": "UniProtKB:B1AL46",
  "term_label": "Unknown molecular function",
  "term_id": "UNKNOWN:0001",
  "gene_name": "NUT family member 2E"
}